{
  "gene_name": "Long-chain fatty acid transport protein 2",
  "gene": "UniProtKB:O14975",
  "term_label": "plasma membrane",
  "term_id": "GO:0005886",
  "gene_symbol": "SLC27A2"
}